{
  "gene": "UniProtKB:P22003",
  "term_id": "GO:0007507",
  "gene_symbol": "BMP5",
  "gene_name": "Bone morphogenetic protein 5",
  "term_label": "heart development"
}